{
  "gene": "UniProtKB:Q96BW1",
  "term_id": "GO:0061769",
  "gene_symbol": "UPRT",
  "term_label": "nicotinate riboside kinase activity",
  "gene_name": "Uracil phosphoribosyltransferase homolog"
}